pyrimidine dimer DNA N-glycosylase activity [GO:0000704] (molecular function) Relationships: is a type of DNA N-glycosylase activity [GO:0019104] References: PMID:9224623 Sources: GOC:elh Definition: Catalysis of the removal of pyrimidine dimers by removing the 5' pyrimidine of the dimer by cleaving the N-C1' glycosidic bond between the 5' pyrimidine of the dimer and the deoxyribose sugar. The reaction releases the 5' pyrimidine of the dimer and leaves an apurinic (AP) site. The reaction involves the formation of a covalent enzyme substrate intermediate. Release of the enzyme and free base by a beta-elimination or a beta, gamma-elimination mechanism results in the cleavage of the DNA backbone 3' of the apyrimidinic (AP) site.